{
  "gene_symbol": "TCAF1",
  "term_id": "GO:0090314",
  "gene": "UniProtKB:Q9Y4C2",
  "gene_name": "TRPM8 channel-associated factor 1",
  "term_label": "positive regulation of protein targeting to membrane"
}